{
  "term_label": "bicellular tight junction",
  "gene": "UniProtKB:P56856",
  "gene_name": "Claudin-18",
  "gene_symbol": "CLDN18",
  "term_id": "GO:0005923"
}